{
  "gene_name": "A disintegrin and metalloproteinase with thrombospondin motifs 20",
  "gene_symbol": "ADAMTS20",
  "gene": "UniProtKB:P59510",
  "term_id": "GO:0004222",
  "term_label": "metalloendopeptidase activity"
}